{
  "term_label": "GPI-anchor transamidase complex",
  "term_id": "GO:0042765",
  "gene_name": "GPI transamidase component PIG-T",
  "gene_symbol": "PIGT",
  "gene": "UniProtKB:Q969N2"
}